SOSS complex [GO:0070876] (cellular component) Relationships: is a type of nuclear protein-containing complex [GO:0140513] Definition: A protein complex that functions downstream of the MRN complex to promote DNA repair and the G2/M checkpoint. The SOSS complex associates with single-stranded DNA at DNA lesions and is composed of SOSS-B (SOSS-B1/OBFC2B or SOSS-B2/OBFC2A), SOSS-A/INTS3 and SOSS-C/C9orf80. References: PMID:19683501